androst-4-ene-3,17-dione monooxygenase activity [GO:0047096] (molecular function) Relationships: is a type of steroid 17-alpha-monooxygenase activity [GO:0004508] Definition: Catalysis of the reaction: AH(2) + androst-4-ene-3,17-dione + O2 = A + H2O + testololactone. Also known as: 4-androstene-3,17-dione monooxygenase activity, androstene-3,17-dione hydroxylase activity, androst-4-ene-3,17-dione 17-oxidoreductase activity, androst-4-ene-3,17-dione hydroxylase activity, androst-4-ene-3,17-dione-hydrogen-donor:oxygen oxidoreductase (13-hydroxylating, lactonizing), androstenedione monooxygenase activity Sources: EC:1.14.99.12, RHEA:22696